{
  "term_id": "GO:0030008",
  "gene_symbol": "TRAPPC12",
  "term_label": "TRAPP complex",
  "gene": "UniProtKB:Q8WVT3",
  "gene_name": "Trafficking protein particle complex subunit 12"
}